{
  "gene_symbol": "TMEM94",
  "gene": "UniProtKB:Q12767",
  "gene_name": "Transmembrane protein 94",
  "term_label": "magnesium ion transport from cytosol to endoplasmic reticulum",
  "term_id": "GO:0160176"
}